cysteine-type endopeptidase regulator activity involved in apoptotic process [GO:0043028] (molecular function) References: PMID:14744432 Sources: GOC:jl, GOC:mtg_apoptosis, Wikipedia:Caspase Definition: Binds to and modulates the activity of a cysteine-type endopeptidase involved in the apoptotic process. Subtypes: cysteine-type endopeptidase activator activity involved in apoptotic process [GO:0008656], cysteine-type endopeptidase inhibitor activity involved in apoptotic process [GO:0043027] Relationships: is a type of enzyme regulator activity [GO:0030234] Also known as: caspase regulator activity